{
  "term_label": "pyridoxal phosphate binding",
  "gene_name": "Serine hydroxymethyltransferase, mitochondrial",
  "gene": "UniProtKB:P34897",
  "term_id": "GO:0030170",
  "gene_symbol": "SHMT2"
}